{
  "term_id": "GO:0031110",
  "gene_symbol": "MAPRE2",
  "gene_name": "Microtubule-associated protein RP_EB family member 2",
  "term_label": "regulation of microtubule polymerization or depolymerization",
  "gene": "UniProtKB:Q15555"
}